regulation of nucleotide-binding domain, leucine rich repeat containing receptor signaling pathway [GO:0070424] (biological process) Subtypes: negative regulation of nucleotide-binding domain, leucine rich repeat containing receptor signaling pathway [GO:0070425], positive regulation of nucleotide-binding domain, leucine rich repeat containing receptor signaling pathway [GO:0070426], regulation of nucleotide-binding oligomerization domain containing 1 signaling pathway [GO:0070428], regulation of nucleotide-binding oligomerization domain containing 2 signaling pathway [GO:0070432] Sources: GOC:add Definition: Any process that modulates the frequency, rate, or extent of a nucleotide-binding domain, leucine rich repeat containing receptor signaling pathway (NLR) pathway. Also known as: regulation of NOD signaling pathway, regulation of nucleotide-binding oligomerization domain containing signaling pathway, regulation of nucleotide-binding oligomerization domain containing signalling pathway Relationships: is a type of regulation of cytoplasmic pattern recognition receptor signaling pathway [GO:0039531]; RO_0002211 nucleotide-binding domain, leucine rich repeat containing receptor signaling pathway [GO:0035872]